{
  "term_label": "brush border",
  "gene": "UniProtKB:Q9UBC5",
  "term_id": "GO:0005903",
  "gene_name": "Unconventional myosin-Ia",
  "gene_symbol": "MYO1A"
}